{
  "gene": "UniProtKB:Q8WUR7",
  "term_id": "UNKNOWN:0001",
  "gene_name": "UPF0235 protein C15orf40",
  "gene_symbol": "C15orf40",
  "term_label": "Unknown molecular function"
}